{
  "term_label": "histone binding",
  "gene_symbol": "SBNO1",
  "gene": "UniProtKB:A3KN83",
  "term_id": "GO:0042393",
  "gene_name": "Protein strawberry notch homolog 1"
}